negative regulation of PERK-mediated unfolded protein response [GO:1903898] (biological process) Definition: Any process that stops, prevents or reduces the frequency, rate or extent of the PERK-mediated unfolded protein response. Relationships: is a type of negative regulation of endoplasmic reticulum unfolded protein response [GO:1900102]; is a type of regulation of PERK-mediated unfolded protein response [GO:1903897]; negatively regulates PERK-mediated unfolded protein response [GO:0036499] References: PMID:22013210 Sources: GOC:PARL, GOC:TermGenie, GOC:bf, GO_REF:0000058 Also known as: down regulation of PERK branch of UPR, down regulation of PERK-mediated unfolded protein response, down regulation of PKR-like ER kinase signal transduction, down regulation of UPR signaling by PERK stress sensor, down regulation of endoplasmic reticulum unfolded protein response; PERK signaling, down-regulation of PERK branch of UPR, down-regulation of PERK-mediated unfolded protein response, down-regulation of PKR-like ER kinase signal transduction, down-regulation of UPR signaling by PERK stress sensor, down-regulation of endoplasmic reticulum unfolded protein response; PERK signaling, downregulation of PERK branch of UPR, downregulation of PERK-mediated unfolded protein response, downregulation of PKR-like ER kinase signal transduction, downregulation of UPR signaling by PERK stress sensor, downregulation of endoplasmic reticulum unfolded protein response; PERK signaling, negative regulation of PERK branch of UPR, negative regulation of PKR-like ER kinase signal transduction, negative regulation of UPR signaling by PERK stress sensor, negative regulation of endoplasmic reticulum unfolded protein response; PERK signaling, inhibition of PERK branch of UPR, inhibition of PERK-mediated unfolded protein response, inhibition of PKR-like ER kinase signal transduction, inhibition of UPR signaling by PERK stress sensor, inhibition of endoplasmic reticulum unfolded protein response; PERK signaling, down regulation of PERK signaling in response to endoplasmic reticulum stress, down-regulation of PERK signaling in response to endoplasmic reticulum stress, downregulation of PERK signaling in response to endoplasmic reticulum stress, inhibition of PERK signaling in response to endoplasmic reticulum stress, negative regulation of EIF2AK3-mediated unfolded protein response, negative regulation of PERK signaling in response to endoplasmic reticulum stress